{
  "term_id": "GO:0045202",
  "gene_name": "Histamine H4 receptor",
  "gene_symbol": "HRH4",
  "term_label": "synapse",
  "gene": "UniProtKB:Q9H3N8"
}